{
  "gene_symbol": "CHD5",
  "term_label": "ATP hydrolysis activity",
  "gene_name": "Chromodomain-helicase-DNA-binding protein 5",
  "gene": "UniProtKB:Q8TDI0",
  "term_id": "GO:0016887"
}